{
  "term_label": "Unknown molecular function",
  "gene_name": "Uncharacterized protein",
  "term_id": "UNKNOWN:0001",
  "gene": "UniProtKB:A0A8V8TND5",
  "gene_symbol": "A0A8V8TND5"
}